{
  "gene_name": "HLA class II histocompatibility antigen, DR beta 5 chain",
  "term_id": "GO:0005765",
  "term_label": "lysosomal membrane",
  "gene_symbol": "HLA-DRB5",
  "gene": "UniProtKB:Q30154"
}